{
  "gene_symbol": "KHDRBS2",
  "gene": "UniProtKB:Q5VWX1",
  "term_label": "nucleus",
  "term_id": "GO:0005634",
  "gene_name": "KH domain-containing, RNA-binding, signal transduction-associated protein 2"
}